{
  "gene": "UniProtKB:P01100",
  "term_label": "DNA-binding transcription factor activity, RNA polymerase II-specific",
  "gene_name": "Protein c-Fos",
  "term_id": "GO:0000981",
  "gene_symbol": "FOS"
}